{
  "gene_name": "Serine-rich single-pass membrane protein 1",
  "term_id": "UNKNOWN:0003",
  "gene": "UniProtKB:Q8WWF3",
  "term_label": "Unknown cellular component",
  "gene_symbol": "SSMEM1"
}